{
  "gene_name": "Transmembrane emp24 domain-containing protein 9",
  "gene_symbol": "TMED9",
  "term_id": "GO:0005793",
  "term_label": "endoplasmic reticulum-Golgi intermediate compartment",
  "gene": "UniProtKB:Q9BVK6"
}